intracellularly cAMP-activated cation channel activity [GO:0005222] (molecular function) Relationships: is a type of GO:0005221 Also known as: HCN channel activity, hyperpolarization-activated cyclic nucleotide-gated channel activity, intracellular 3',5' cAMP activated cation channel activity, intracellular 3',5'-cAMP activated cation channel activity, intracellular adenosine 3',5'-cyclophosphate activated cation channel activity, intracellular cAMP activated cation channel activity, intracellular cAMP-activated cation channel activity, intracellular cyclic AMP activated cation channel activity Sources: GOC:mtg_transport Subtypes: GO:0140232, GO:0140233 Definition: Enables the transmembrane transfer of a cation by a channel that opens when intracellular cAMP has been bound by the channel complex or one of its constituent parts.